{
  "gene": "UniProtKB:O75943",
  "gene_symbol": "RAD17",
  "term_id": "GO:0031389",
  "term_label": "Rad17 RFC-like complex",
  "gene_name": "Cell cycle checkpoint protein RAD17"
}